establishment of cell polarity involved in gastrulation cell migration [GO:0003379] (biological process) Definition: The specification and formation of anisotropic intracellular organization that contributes to the self-propelled directed movement of an ameboid cell taking part in gastrulation. Subtypes: establishment of cell polarity involved in mesendodermal cell migration [GO:0003369] Relationships: is a type of establishment of cell polarity involved in ameboidal cell migration [GO:0003365]; BFO_0000050 cell migration involved in gastrulation [GO:0042074] Sources: GOC:ascb_2009, GOC:dph, GOC:tb